{
  "gene_symbol": "OVOL2",
  "gene": "UniProtKB:Q9BRP0",
  "term_label": "nucleus",
  "gene_name": "Transcription factor Ovo-like 2",
  "term_id": "GO:0005634"
}